{
  "gene_symbol": "STARD10",
  "gene": "UniProtKB:Q9Y365",
  "term_label": "microvillus",
  "term_id": "GO:0005902",
  "gene_name": "START domain-containing protein 10"
}